RSF complex [GO:0031213] (cellular component) Definition: An ISWI complex that contains an ATPase subunit of the ISWI family (SNF2H in mammals) and an RSF1 homolog. It mediates nucleosome deposition and generates regularly spaced nucleosome arrays. In mammals, RSF is involved in regulation of transcription from RNA polymerase II promoters). Also known as: remodeling and spacing factor complex Relationships: is a type of GO:0031010 References: PMID:12972596, PMID:15284901, PMID:16568949, PMID:21810179 Sources: GOC:krc